{
  "gene": "UniProtKB:Q4LDR2",
  "term_id": "UNKNOWN:0003",
  "term_label": "Unknown cellular component",
  "gene_name": "Cortexin-3",
  "gene_symbol": "CTXN3"
}